{
  "term_id": "GO:0005615",
  "gene_name": "Protein Wnt-10b",
  "gene_symbol": "WNT10B",
  "gene": "UniProtKB:O00744",
  "term_label": "extracellular space"
}